{
  "term_id": "UNKNOWN:0001",
  "gene": "UniProtKB:P0DPQ3",
  "gene_name": "Proline-rich protein 20G",
  "gene_symbol": "PRR20G",
  "term_label": "Unknown molecular function"
}